{
  "term_id": "UNKNOWN:0003",
  "gene": "UniProtKB:P0DQW1",
  "gene_name": "Small integral membrane protein 46",
  "gene_symbol": "SMIM46",
  "term_label": "Unknown cellular component"
}